{
  "gene_name": "Forkhead box protein E3",
  "term_id": "GO:0000981",
  "gene_symbol": "FOXE3",
  "gene": "UniProtKB:Q13461",
  "term_label": "DNA-binding transcription factor activity, RNA polymerase II-specific"
}